regulation of meiotic cell cycle phase transition [GO:1901993] (BP) Subtypes: regulation of exit from meiosis [GO:0106060], regulation of G2/MI transition of meiotic cell cycle [GO:0110030], negative regulation of meiotic cell cycle phase transition [GO:1901994], GO:1901995, regulation of metaphase/anaphase transition of meiotic cell cycle [GO:1902102] References: PMID:22841721 Sources: GOC:TermGenie, GOC:mtg_cell_cycle Definition: Any process that modulates the frequency, rate or extent of meiotic cell cycle phase transition. Also known as: regulation of cell cycle transition, meiotic cell cycle control Relationships: is a type of regulation of cell cycle phase transition [GO:1901987]; is a type of regulation of reproductive process [GO:2000241]; regulates meiotic cell cycle phase transition [GO:0044771]